{
  "gene": "UniProtKB:O75030",
  "gene_name": "Microphthalmia-associated transcription factor",
  "term_id": "GO:0006357",
  "term_label": "regulation of transcription by RNA polymerase II",
  "gene_symbol": "MITF"
}